{
  "gene_symbol": "OR2T8",
  "gene_name": "Olfactory receptor 2T8",
  "term_label": "plasma membrane",
  "term_id": "GO:0005886",
  "gene": "UniProtKB:A6NH00"
}